peptide amidation [GO:0001519] (biological process) Definition: The posttranslational conversion of C-terminal glycine-extended peptides to C-terminal alpha-amidated peptides. Occurs to over half of all peptide hormones to give bioactive peptides. This is a two step process catalyzed by a peptidyl-glycine alpha-hydroxylating monooxygenase and a peptidyl-alpha-hydroxyglycine alpha-amidating lyase. In some organisms, this process is catalyzed by two separate enzymes, whereas in higher organisms, one polypeptide catalyzes both reactions. References: PMID:11028916 Relationships: is a type of GO:0031179